TFIIE-class transcription factor complex binding [GO:0001095] (molecular function) Relationships: is a type of RNA polymerase II general transcription initiation factor binding [GO:0001091]; is a type of protein-containing complex binding [GO:0044877] Also known as: TFIIE-class transcription factor binding Definition: Binding to a general RNA polymerase II transcription factor belonging to the TFIIE complex, one of the factors involved in formation of the preinitiation complex (PIC) by RNA polymerase II. References: PMID:16858867 Sources: GOC:krc